{
  "term_label": "mitochondrial ribosome",
  "gene_symbol": "MRPL20",
  "gene": "UniProtKB:Q9BYC9",
  "gene_name": "Large ribosomal subunit protein bL20m",
  "term_id": "GO:0005761"
}